UDP-glucuronate metabolic process [GO:0046398] (biological process) Definition: The chemical reactions and pathways involving UDP-glucuronate, a substance composed of glucuronic acid in glycosidic linkage with uridine diphosphate. Sources: GOC:ai Subtypes: UDP-glucuronate biosynthetic process [GO:0006065] Relationships: is a type of nucleotide-sugar metabolic process [GO:0009225]; is a type of carboxylic acid metabolic process [GO:0019752] Also known as: UDP-glucuronate metabolism